{
  "gene_symbol": "CNGA4",
  "term_id": "GO:0098655",
  "term_label": "monoatomic cation transmembrane transport",
  "gene": "UniProtKB:Q8IV77",
  "gene_name": "Cyclic nucleotide-gated cation channel alpha-4"
}